glycine betaine biosynthetic process [GO:0031456] (BP) Relationships: is a type of amino-acid betaine biosynthetic process [GO:0006578] Subtypes: glycine betaine biosynthetic process from choline [GO:0019285], glycine betaine biosynthetic process from glycine [GO:0019286] Sources: GOC:mah Definition: The chemical reactions and pathways resulting in the formation of glycine betaine, N-trimethylglycine. Also known as: N-trimethylglycine biosynthesis, N-trimethylglycine biosynthetic process, glycine betaine anabolism, glycine betaine biosynthesis, glycine betaine formation, glycine betaine synthesis